{
  "gene": "UniProtKB:Q9P225",
  "term_id": "GO:0030286",
  "gene_name": "Dynein axonemal heavy chain 2",
  "term_label": "dynein complex",
  "gene_symbol": "DNAH2"
}